NAD+-protein-arginine ADP-ribosyltransferase activity [GO:0106274] (molecular function) Sources: RHEA:19149 Definition: Catalysis of the reaction: L-arginyl-[protein] + NAD+ = H+ + (ADP-D-ribosyl)-L-arginyl-[protein] + nicotinamide. Relationships: is a type of GO:1990404 Also known as: ADP-ribosyltransferase activity, NAD(P)+-protein-arginine ADP-ribosyltransferase activity, NADP+-protein-arginine ADP-ribosyltransferase activity, mono(ADP-ribosyl)transferase activity, NAD(+):L-arginine ADP-D-ribosyltransferase activity, NAD(P)(+)--arginine ADP-ribosyltransferase activity, NAD(P)+:L-arginine ADP-D-ribosyltransferase activity, peptidyl-arginine ADP-ribosylation activity, protein-arginine ADP-ribosyltransferase activity, NAD(P)+:protein-L-arginine ADP-D-ribosyltransferase activity